negative regulation of nurse cell apoptotic process [GO:0045849] (biological process) Definition: Any process that stops, prevents, or reduces the frequency, rate or extent of nurse cell apoptotic process. Relationships: is a type of regulation of nurse cell apoptotic process [GO:0045477]; is a type of negative regulation of apoptotic process involved in development [GO:1904746]; is_a GO:2000242; negatively regulates nurse cell apoptotic process [GO:0045476] Sources: GOC:go_curators, GOC:mtg_apoptosis Also known as: down regulation of nurse cell apoptosis, down-regulation of nurse cell apoptosis, downregulation of nurse cell apoptosis, inhibition of nurse cell apoptosis, negative regulation of nurse cell apoptosis